{
  "term_label": "autophagosome membrane",
  "gene_symbol": "STX17",
  "term_id": "GO:0000421",
  "gene": "UniProtKB:P56962",
  "gene_name": "Syntaxin-17"
}